{
  "gene_name": "Collagen alpha-1(XX) chain",
  "gene_symbol": "COL20A1",
  "term_id": "UNKNOWN:0003",
  "gene": "UniProtKB:Q9P218",
  "term_label": "Unknown cellular component"
}